{
  "term_label": "positive regulation of cholesterol efflux",
  "gene_name": "Palmitoyltransferase ZDHHC8",
  "gene_symbol": "ZDHHC8",
  "gene": "UniProtKB:Q9ULC8",
  "term_id": "GO:0010875"
}